purine deoxyribonucleotide interconversion [GO:0015952] (biological process) Relationships: is a type of purine deoxyribonucleotide metabolic process [GO:0009151]; is a type of purine nucleotide interconversion [GO:0015950] Sources: GOC:mah, ISBN:0306444747, ISBN:0471394831 Definition: The chemical reactions and pathways by which a purine deoxyribonucleotide is synthesized from another purine deoxyribonucleotide.